{
  "term_label": "cellular response to amino acid starvation",
  "term_id": "GO:0034198",
  "gene_symbol": "KPTN",
  "gene_name": "KICSTOR complex protein kaptin",
  "gene": "UniProtKB:Q9Y664"
}